{
  "gene_name": "Olfactory receptor 1D2",
  "gene": "UniProtKB:P34982",
  "term_label": "olfactory receptor activity",
  "gene_symbol": "OR1D2",
  "term_id": "GO:0004984"
}